{
  "gene_symbol": "IFNA6",
  "gene_name": "Interferon alpha-6",
  "term_id": "GO:0006959",
  "term_label": "humoral immune response",
  "gene": "UniProtKB:P05013"
}